{
  "term_label": "transcription cis-regulatory region binding",
  "gene_name": "Zinc finger protein 600",
  "term_id": "GO:0000976",
  "gene_symbol": "ZNF600",
  "gene": "UniProtKB:Q6ZNG1"
}